{
  "term_id": "GO:0001228",
  "gene": "UniProtKB:P35716",
  "gene_name": "Transcription factor SOX-11",
  "gene_symbol": "SOX11",
  "term_label": "DNA-binding transcription activator activity, RNA polymerase II-specific"
}